{
  "term_id": "GO:0030198",
  "gene_symbol": "COL4A6",
  "gene_name": "Collagen alpha-6(IV) chain",
  "gene": "UniProtKB:Q14031",
  "term_label": "extracellular matrix organization"
}